rod bipolar cell differentiation [GO:1904389] (biological process) Relationships: is a type of retinal bipolar neuron differentiation [GO:0060040] Definition: The process in which a relatively unspecialized cell acquires the specialized features of a rod bipolar cell. References: PMID:16914133 Sources: GOC:TermGenie, GO_REF:0000086